sodium channel regulator activity [GO:0017080] (molecular function) Subtypes: GO:0019871 Relationships: is a type of ion channel regulator activity [GO:0099106]; regulates GO:0005272 Sources: GOC:mah Definition: Binds to and modulates the activity of a sodium channel.